{
  "gene": "UniProtKB:Q86YP4",
  "gene_symbol": "GATAD2A",
  "gene_name": "Transcriptional repressor p66-alpha",
  "term_id": "GO:0000122",
  "term_label": "negative regulation of transcription by RNA polymerase II"
}